{
  "gene_name": "Ermin",
  "gene": "UniProtKB:Q8TAM6",
  "gene_symbol": "ERMN",
  "term_label": "myelin sheath",
  "term_id": "GO:0043209"
}